{
  "gene_name": "Serine_threonine-protein kinase WNK1",
  "term_id": "GO:0090263",
  "gene_symbol": "WNK1",
  "gene": "UniProtKB:Q9H4A3",
  "term_label": "positive regulation of canonical Wnt signaling pathway"
}